{
  "term_id": "GO:0005216",
  "gene": "UniProtKB:P81605",
  "gene_symbol": "DCD",
  "term_label": "monoatomic ion channel activity",
  "gene_name": "Dermcidin"
}